{
  "gene_name": "Hepatocyte nuclear factor 1-beta",
  "gene": "UniProtKB:P35680",
  "term_id": "GO:0006357",
  "term_label": "regulation of transcription by RNA polymerase II",
  "gene_symbol": "HNF1B"
}